positive regulation of placenta blood vessel development [GO:0110080] (biological process) References: PMID:27748453 Sources: GOC:BHF, GOC:BHF_miRNA, GOC:rph Definition: Any process that activates or increases the frequency, rate or extent of placenta blood vessel development. Relationships: is a type of GO:0051094; is a type of regulation of placenta blood vessel development [GO:0110079]; RO_0002213 placenta blood vessel development [GO:0060674]